{
  "gene_name": "Stromal cell-derived factor 1",
  "gene_symbol": "CXCL12",
  "term_id": "GO:0060326",
  "gene": "UniProtKB:P48061",
  "term_label": "cell chemotaxis"
}